positive regulation of cytokine-mediated signaling pathway [GO:0001961] (biological process) Sources: GOC:hjd Also known as: positive regulation of cytokine and chemokine mediated signaling pathway, positive regulation of cytokine mediated signaling pathway, positive regulation of cytokine mediated signalling pathway, up regulation of cytokine mediated signaling pathway, up-regulation of cytokine mediated signaling pathway, upregulation of cytokine mediated signaling pathway, activation of cytokine mediated signaling pathway, stimulation of cytokine mediated signaling pathway Definition: Any process that activates or increases the frequency, rate or extent of a cytokine mediated signaling pathway. Relationships: is a type of regulation of cytokine-mediated signaling pathway [GO:0001959]; is a type of positive regulation of signal transduction [GO:0009967]; is a type of positive regulation of response to cytokine stimulus [GO:0060760]; positively regulates cytokine-mediated signaling pathway [GO:0019221] Subtypes: GO:0060335, positive regulation of type I interferon-mediated signaling pathway [GO:0060340], positive regulation of chemokine-mediated signaling pathway [GO:0070101], positive regulation of interleukin-6-mediated signaling pathway [GO:0070105], positive regulation of interleukin-27-mediated signaling pathway [GO:0070109], GO:0070760, positive regulation of Kit signaling pathway [GO:1900236], GO:1902207, GO:1902213, GO:1902216, positive regulation of macrophage colony-stimulating factor signaling pathway [GO:1902228], positive regulation of tumor necrosis factor-mediated signaling pathway [GO:1903265], positive regulation of interleukin-17-mediated signaling pathway [GO:1903883], positive regulation of macrophage migration inhibitory factor signaling pathway [GO:2000448], positive regulation of interleukin-18-mediated signaling pathway [GO:2000494], positive regulation of interleukin-1-mediated signaling pathway [GO:2000661]